glucose-1,6-bisphosphate synthase activity [GO:0047933] (molecular function) Also known as: 3-phospho-D-glyceroyl-phosphate:D-glucose-1-phosphate 6-phosphotransferase activity, 3-phospho-D-glyceroyl-phosphate:alpha-D-glucose-1-phosphate 6-phosphotransferase activity, glucose 1,6-diphosphate synthase activity, glucose-1,6-bisphosphate synthetase activity Sources: EC:2.7.1.106, RHEA:16769 Relationships: is a type of kinase activity [GO:0016301]; is a type of GO:0016773 Definition: Catalysis of the reaction: 3-phospho-D-glyceroyl phosphate + alpha-D-glucose 1-phosphate = 3-phospho-D-glycerate + alpha-D-glucose 1,6-bisphosphate + H+.